{
  "gene": "UniProtKB:Q14094",
  "gene_symbol": "CCNI",
  "term_label": "nucleus",
  "term_id": "GO:0005634",
  "gene_name": "Cyclin-I"
}